{
  "gene_name": "Putative uncharacterized protein FLJ46641",
  "gene": "UniProtKB:Q6ZR54",
  "term_label": "Unknown cellular component",
  "gene_symbol": "Q6ZR54",
  "term_id": "UNKNOWN:0003"
}